{
  "gene_name": "Neuronal migration protein doublecortin",
  "term_label": "Unknown cellular component",
  "gene": "UniProtKB:O43602",
  "gene_symbol": "DCX",
  "term_id": "UNKNOWN:0003"
}